{
  "gene_name": "Guanine nucleotide-binding protein G(s) subunit alpha isoforms XLas",
  "gene": "UniProtKB:Q5JWF2",
  "term_label": "mu-type opioid receptor binding",
  "gene_symbol": "GNAS",
  "term_id": "GO:0031852"
}